F-box domain binding [GO:1990444] (molecular function) References: PMID:12628165 Sources: GOC:PARL, GOC:bf, InterPro:IPR001810 Definition: Binding to an F-box domain of a protein. Relationships: is_a GO:0019904